{
  "gene_symbol": "SORBS2",
  "gene": "UniProtKB:O94875",
  "term_label": "Notch signaling pathway",
  "gene_name": "Sorbin and SH3 domain-containing protein 2",
  "term_id": "GO:0007219"
}